regulation of podosome assembly [GO:0071801] (biological process) Note: Note that the assembly is regulated by several small GTPases of the Rab and Rho families. Definition: Any process that modulates the frequency, rate or extent of podosome assembly. Subtypes: negative regulation of podosome assembly [GO:0071802], positive regulation of podosome assembly [GO:0071803] Relationships: is a type of regulation of protein-containing complex assembly [GO:0043254]; is a type of regulation of organelle assembly [GO:1902115]; regulates GO:0071800 Sources: GOC:mah, GOC:sl